{
  "gene_name": "Pleckstrin homology domain-containing family G member 7",
  "term_label": "guanyl-nucleotide exchange factor activity",
  "gene": "UniProtKB:Q6ZR37",
  "term_id": "GO:0005085",
  "gene_symbol": "PLEKHG7"
}